ISG15 activating enzyme activity [GO:0019782] (molecular function) Relationships: is a type of ubiquitin-like modifier activating enzyme activity [GO:0008641] Sources: GOC:mah Definition: Catalysis of the activation of the small ubiquitin-related modifier ISG15, through the formation of an ATP-dependent high-energy thiolester bond. Also known as: UBE1L